{
  "term_id": "GO:0000977",
  "gene_symbol": "ISX",
  "gene_name": "Intestine-specific homeobox",
  "term_label": "RNA polymerase II transcription regulatory region sequence-specific DNA binding",
  "gene": "UniProtKB:Q2M1V0"
}